{
  "gene": "UniProtKB:Q5T601",
  "term_id": "GO:0005886",
  "term_label": "plasma membrane",
  "gene_name": "Adhesion G-protein coupled receptor F1",
  "gene_symbol": "ADGRF1"
}